{
  "gene": "UniProtKB:P32519",
  "term_label": "regulation of transcription by RNA polymerase II",
  "term_id": "GO:0006357",
  "gene_name": "ETS-related transcription factor Elf-1",
  "gene_symbol": "ELF1"
}